pyramidal neuron differentiation [GO:0021859] (biological process) Definition: The process in which a neuroblast or one of its progeny commits to a pyramidal neuron fate, migrates from the ventricular zone to the appropriate layer in the cortex and develops into a mature neuron. Subtypes: hippocampal pyramidal neuron differentiation [GO:0097432], Meynert cell differentiation [GO:1905270] Also known as: projection neuron differentiation Relationships: is a type of central nervous system neuron differentiation [GO:0021953] Sources: GOC:cls, GOC:dgh, GOC:dph, GOC:jid, GO_REF:0000021